{
  "term_id": "GO:0005634",
  "term_label": "nucleus",
  "gene": "UniProtKB:P35659",
  "gene_symbol": "DEK",
  "gene_name": "Protein DEK"
}